{
  "gene_name": "Iroquois-class homeodomain protein IRX-3",
  "term_id": "GO:0000978",
  "gene": "UniProtKB:P78415",
  "term_label": "RNA polymerase II cis-regulatory region sequence-specific DNA binding",
  "gene_symbol": "IRX3"
}